{
  "term_id": "GO:0032438",
  "term_label": "melanosome organization",
  "gene": "UniProtKB:P57729",
  "gene_name": "Ras-related protein Rab-38",
  "gene_symbol": "RAB38"
}